{
  "gene": "UniProtKB:Q5VXJ0",
  "term_label": "lipase activity",
  "gene_symbol": "LIPK",
  "term_id": "GO:0016298",
  "gene_name": "Lipase member K"
}